{
  "gene_name": "NFIL3 like protein",
  "gene": "UniProtKB:A0A5F9ZHS7",
  "gene_symbol": "NFILZ",
  "term_id": "UNKNOWN:0001",
  "term_label": "Unknown molecular function"
}